DNA-3-methyladenine glycosylase activity [GO:0008725] (molecular function) Definition: Catalysis of the reaction: DNA containing 3-methyladenine + H2O = DNA with abasic site + 3-methyladenine. This reaction is the hydrolysis of DNA by cleavage of the N-C1' glycosidic bond between the damaged DNA 3-methyladenine and the deoxyribose sugar to remove the 3-methyladenine, leaving an abasic site. References: PMID:10872450, PMID:9224623 Sources: EC:3.2.2.20, GOC:elh Also known as: DNA-3-methyladenine glycosylase I activity, 3-methyladenine DNA glycosylase I, DNA glycosidase I activity, DNA-3-methyladenine glycosidase I activity, deoxyribonucleate 3-methyladenine glycosidase I Relationships: is a type of GO:0043733